Herring body [GO:1990623] (cellular component) Relationships: is a type of axon terminus [GO:0043679] Definition: The dilated terminal portions of neurosecretory axons constituting the hypothalamohypophyseal tract, found in close proximity to sinusoidal capillaries in the posterior pituitary. Herring bodies consist of aggregates of membrane-bound neurosecretory vesicles where oxytocin or antidiuretic hormone (ADH) are stored prior to release. Each Herring body also contains ATP and either neurophysin I or neurophysin II which bind to oxytocin and ADH, respectively. Sources: ISBN:0199652473, Wikipedia:Herring_bodies Also known as: neurosecretory body